cellular response to sodium dodecyl sulfate [GO:0072707] (biological process) Sources: GOC:mah Also known as: cellular response to SDS Definition: Any process that results in a change in state or activity of a cell (in terms of movement, secretion, enzyme production, gene expression, etc.) as a result of a sodium dodecyl sulfate (SDS) stimulus. Relationships: is a type of GO:0072706; is a type of cellular response to oxygen-containing compound [GO:1901701]